spore encystment [GO:0075214] (biological process) Definition: The physiological, developmental and morphological changes that occur in a symbiont spore during the process of its encystment. Encystment means to enter a state of essentially suspended animation in which the spore is protected by an outer coating and remains immobile and inactive until favorable conditions for growth occur again. The host is defined as the larger of the organisms involved in a symbiotic interaction. Sources: GOC:kmv, GOC:pamgo_curators Also known as: spore encystment on host Relationships: is a type of dormancy process [GO:0022611]; is a type of cell development [GO:0048468] Subtypes: zoospore encystment on host [GO:0075218] Regulation: RO_0002211 by GO:0075215; positively regulated by positive regulation of spore encystment on host [GO:0075216]; negatively regulated by GO:0075217